{
  "gene_symbol": "LGALS3",
  "gene_name": "Galectin-3",
  "term_id": "GO:0048245",
  "term_label": "eosinophil chemotaxis",
  "gene": "UniProtKB:P17931"
}